N-acylneuraminate cytidylyltransferase activity [GO:0008781] (molecular function) Definition: Catalysis of the reaction: CTP + N-acylneuraminate = diphosphate + CMP-N-acylneuraminate. Also known as: CTP:N-acylneuraminate cytidylyltransferase activity, CMP-N-acetylneuraminate synthase activity, CMP-N-acetylneuraminate synthetase activity, CMP-N-acetylneuraminic acid synthase activity, CMP-N-acetylneuraminic acid synthetase activity, CMP-NANA synthetase activity, CMP-Neu5Ac synthetase activity, CMP-NeuAc synthetase activity, CMP-NeuNAc synthetase activity, CMP-sialate diphosphorylase activity, CMP-sialate pyrophosphorylase activity, CMP-sialate synthase activity, CMP-sialate synthetase activity, CMP-sialic acid synthetase activity, CMP-sialic synthetase activity, acetylneuraminate cytidylyltransferase activity, acylneuraminate cytidyltransferase activity, cytidine 5'-monophospho-N-acetylneuraminic acid synthetase activity, cytidine 5'-monophosphosialic acid synthetase activity, cytidine 5-monophosphate N-acetylneuraminic acid synthetase activity, cytidine monophosphoacetylneuraminic synthetase activity, cytidine monophosphosialate pyrophosphorylase activity, cytidine monophosphosialate synthetase activity, cytidine monophosphosialic acid synthetase activity Sources: EC:2.7.7.43 Relationships: is a type of cytidylyltransferase activity [GO:0070567]